{
  "term_label": "olfactory receptor activity",
  "term_id": "GO:0004984",
  "gene": "UniProtKB:Q5JRS4",
  "gene_symbol": "OR10J3",
  "gene_name": "Olfactory receptor 10J3"
}